regulation of positive chemotaxis to cAMP by chlorinated alkylphenone [GO:0061119] (biological process) Definition: Any process that modulates the rate, frequency, or extent of directed movement of a motile cell or organism up a concentration gradient of 3',5'-cAMP by the action of a chlorinated alkylphenone. An alkylphenone is an aromatic polyketide with methyl and chlorine substitutions. References: PMID:19684855 Sources: GOC:dph Relationships: is a type of GO:0061118 Subtypes: GO:0061120, regulation of positive chemotaxis to cAMP by DIF-2 [GO:0061121], positive regulation of positive chemotaxis to cAMP by chlorinated alkylphenone [GO:0061124], negative regulation of positive chemotaxis to cAMP by chlorinated alkylphenone [GO:0061125]